{
  "term_id": "GO:0005886",
  "gene": "UniProtKB:Q9UBG0",
  "gene_name": "C-type mannose receptor 2",
  "term_label": "plasma membrane",
  "gene_symbol": "MRC2"
}